{
  "term_id": "UNKNOWN:0001",
  "gene_name": "Protocadherin-23",
  "gene": "UniProtKB:Q6V1P9",
  "term_label": "Unknown molecular function",
  "gene_symbol": "DCHS2"
}